{
  "gene": "UniProtKB:P04181",
  "term_id": "GO:0030170",
  "gene_symbol": "OAT",
  "gene_name": "Ornithine aminotransferase, mitochondrial",
  "term_label": "pyridoxal phosphate binding"
}